{
  "term_id": "GO:0048812",
  "gene": "UniProtKB:O60237",
  "gene_symbol": "PPP1R12B",
  "gene_name": "Protein phosphatase 1 regulatory subunit 12B",
  "term_label": "neuron projection morphogenesis"
}